{
  "gene_name": "Epididymal-specific lipocalin-8",
  "term_label": "Unknown biological process",
  "gene_symbol": "LCN8",
  "term_id": "UNKNOWN:0002",
  "gene": "UniProtKB:Q6JVE9"
}